{
  "gene_symbol": "BRAT1",
  "term_label": "DNA damage response",
  "gene": "UniProtKB:Q6PJG6",
  "gene_name": "BRCA1-associated ATM activator 1",
  "term_id": "GO:0006974"
}